{
  "term_id": "GO:0000978",
  "term_label": "RNA polymerase II cis-regulatory region sequence-specific DNA binding",
  "gene": "UniProtKB:Q06413",
  "gene_name": "Myocyte-specific enhancer factor 2C",
  "gene_symbol": "MEF2C"
}